NAD+-protein-tyrosine ADP-ribosyltransferase activity [GO:0140808] (molecular function) Definition: Catalysis of the reaction: L-tyrosyl-[protein] + NAD+ = H+ + nicotinamide + O-(ADP-D-ribosyl)-L-tyrosyl-[protein]. References: PMID:29954836, PMID:30257210 Sources: RHEA:58236 Relationships: is a type of NAD+-protein mono-ADP-ribosyltransferase activity [GO:1990404]